{
  "term_label": "Unknown biological process",
  "gene_name": "Dynactin subunit 5",
  "term_id": "UNKNOWN:0002",
  "gene": "UniProtKB:Q9BTE1",
  "gene_symbol": "DCTN5"
}